{
  "term_id": "GO:0043186",
  "term_label": "P granule",
  "gene_symbol": "TDRD1",
  "gene_name": "Tudor domain-containing protein 1",
  "gene": "UniProtKB:Q9BXT4"
}